transposable element silencing by siRNA-mediated heterochromatin formation [GO:0141007] (biological process) Also known as: siRNA-mediated retrotransposon silencing by heterochromatin formation Definition: A transposable element silencing mechanism in which a siRNA triggers heterochromatin assembly. Heterochromatin is a chromatin conformation that is refractory to transcription. Relationships: is_a transposable element silencing by heterochromatin formation [GO:0141005]; is a type of siRNA-mediated heterochromatin formation [GO:0141194] References: PMID:36570931